{
  "term_label": "G1/S transition of mitotic cell cycle",
  "gene": "UniProtKB:O96020",
  "gene_name": "G1_S-specific cyclin-E2",
  "term_id": "GO:0000082",
  "gene_symbol": "CCNE2"
}